{
  "gene_name": "Flap endonuclease 1",
  "gene": "UniProtKB:P39748",
  "term_label": "5'-flap endonuclease activity",
  "term_id": "GO:0017108",
  "gene_symbol": "FEN1"
}